{
  "term_id": "GO:0050839",
  "term_label": "cell adhesion molecule binding",
  "gene_symbol": "PTPN11",
  "gene": "UniProtKB:Q06124",
  "gene_name": "Tyrosine-protein phosphatase non-receptor type 11"
}